{
  "gene_symbol": "RRAD",
  "term_id": "GO:0005525",
  "gene_name": "GTP-binding protein RAD",
  "gene": "UniProtKB:P55042",
  "term_label": "GTP binding"
}